{
  "gene_name": "Sulfotransferase 4A1",
  "gene_symbol": "SULT4A1",
  "gene": "UniProtKB:Q9BR01",
  "term_label": "cytoplasm",
  "term_id": "GO:0005737"
}